positive regulation of heterochromatin formation [GO:0031453] (biological process) Definition: Any process that activates or increases the frequency, rate or extent of heterochromatin formation. Also known as: positive regulation of heterochromatin assembly, up regulation of heterochromatin formation, up-regulation of heterochromatin formation, upregulation of heterochromatin formation, activation of heterochromatin formation, stimulation of heterochromatin formation Subtypes: positive regulation of pericentric heterochromatin formation [GO:0090053], GO:0090055, positive regulation of rDNA heterochromatin formation [GO:2000749] Sources: GOC:mah Relationships: is a type of regulation of heterochromatin formation [GO:0031445]; is a type of positive regulation of cellular component biogenesis [GO:0044089]; is a type of positive regulation of chromatin organization [GO:1905269]; positively regulates GO:0031507